{
  "gene": "UniProtKB:Q9Y3A0",
  "gene_symbol": "COQ4",
  "term_id": "GO:0006744",
  "gene_name": "Ubiquinone biosynthesis protein COQ4 homolog, mitochondrial",
  "term_label": "ubiquinone biosynthetic process"
}